axial mesodermal cell differentiation [GO:0048321] (biological process) Definition: The process in which a relatively unspecialized cell acquires specialized features of an axial mesoderm cell. Sources: GOC:dgh Also known as: axial mesoderm cell differentiation Relationships: is a type of GO:0048333; is part of GO:0048320